{
  "gene_symbol": "BAIAP2L1",
  "gene": "UniProtKB:Q9UHR4",
  "term_id": "GO:0051017",
  "term_label": "actin filament bundle assembly",
  "gene_name": "Brain-specific angiogenesis inhibitor 1-associated protein 2-like protein 1"
}